{
  "term_label": "liver development",
  "gene_symbol": "UGT1A9",
  "gene": "UniProtKB:O60656",
  "term_id": "GO:0001889",
  "gene_name": "UDP-glucuronosyltransferase 1A9"
}